{
  "gene_name": "WD repeat-containing protein 35",
  "term_id": "GO:0060271",
  "term_label": "cilium assembly",
  "gene_symbol": "WDR35",
  "gene": "UniProtKB:Q9P2L0"
}